{
  "gene_name": "Bone morphogenetic protein 8B",
  "gene_symbol": "BMP8B",
  "term_label": "BMP signaling pathway",
  "gene": "UniProtKB:P34820",
  "term_id": "GO:0030509"
}